{
  "gene_symbol": "PLPP3",
  "gene_name": "Phospholipid phosphatase 3",
  "term_label": "cell-cell adhesion",
  "gene": "UniProtKB:O14495",
  "term_id": "GO:0098609"
}